cellular response to molecule of fungal origin [GO:0071226] (biological process) Also known as: cellular response to fungus associated molecule Sources: GOC:mah Relationships: is a type of response to molecule of fungal origin [GO:0002238]; is a type of cellular response to biotic stimulus [GO:0071216] Definition: Any process that results in a change in state or activity of a cell (in terms of movement, secretion, enzyme production, gene expression, etc.) as a result of a stimulus by molecules of fungal origin such as chito-octamer oligosaccharide.